{
  "term_id": "UNKNOWN:0002",
  "gene_name": "Putative protein FAM90A12P",
  "gene": "UniProtKB:A8MX19",
  "term_label": "Unknown biological process",
  "gene_symbol": "FAM90A12P"
}